{
  "gene_symbol": "AP2M1",
  "term_label": "synaptic vesicle",
  "term_id": "GO:0008021",
  "gene_name": "AP-2 complex subunit mu",
  "gene": "UniProtKB:Q96CW1"
}